regulation of protein exit from endoplasmic reticulum [GO:0070861] (biological process) Subtypes: negative regulation of protein exit from endoplasmic reticulum [GO:0070862], positive regulation of protein exit from endoplasmic reticulum [GO:0070863], regulation of retrograde protein transport, ER to cytosol [GO:1904152] Definition: Any process that modulates the frequency, rate or extent of the directed movement of proteins from the endoplasmic reticulum. Relationships: is a type of GO:0033157; regulates GO:0032527 Also known as: regulation of protein exit from ER, regulation of protein export from ER, regulation of protein export from endoplasmic reticulum Sources: GOC:mah